endocytosis [GO:0006897] (biological process) Also known as: endocytic import into cell, vesicle endocytosis, plasma membrane invagination, nonselective vesicle endocytosis Relationships: is a type of GO:0016192; is a type of GO:0098657; has part vesicle budding from membrane [GO:0006900]; has part membrane invagination [GO:0010324] Sources: GOC:mah, ISBN:0198506732, ISBN:0716731363, Wikipedia:Endocytosis Subtypes: GO:0006898, pinocytosis [GO:0006907], phagocytosis [GO:0006909], GO:0035037, ubiquitin-dependent endocytosis [GO:0070086], GO:0072584, presynaptic endocytosis [GO:0140238], postsynaptic endocytosis [GO:0140239], GO:0160294 Definition: A vesicle-mediated transport process in which cells take up external materials or membrane constituents by the invagination of a part of the plasma membrane to form a new membrane-bounded vesicle. Regulation: regulated by GO:0030100; negatively regulated by negative regulation of endocytosis [GO:0045806]; positively regulated by positive regulation of endocytosis [GO:0045807]